regulation of cardiac muscle adaptation [GO:0010612] (biological process) Subtypes: GO:0010615, GO:0010616, regulation of cardiac muscle hypertrophy in response to stress [GO:1903242] Definition: Any process that modulates the rate, extent or frequency of the process in which cardiac muscle adapts, with consequent modifications to structural and/or functional phenotypes, in response to a stimulus. Stimuli include contractile activity, loading conditions, substrate supply, and environmental factors. Relationships: is a type of GO:0043502; regulates cardiac muscle adaptation [GO:0014887] Sources: GOC:dph, GOC:tb